positive regulation of cell adhesion molecule production [GO:0060355] (biological process) Definition: Any process that increases the rate, frequency or extent of cell adhesion molecule production. Cell adhesion molecule production is the appearance of a cell adhesion molecule as a result of its biosynthesis or a decrease in its catabolism. Sources: GOC:BHF, GOC:rl Relationships: is_a positive regulation of cellular process [GO:0048522]; is a type of regulation of cell adhesion molecule production [GO:0060353]; RO_0002213 cell adhesion molecule production [GO:0060352]